{
  "gene": "UniProtKB:Q9UNH6",
  "term_label": "early endosome",
  "gene_symbol": "SNX7",
  "term_id": "GO:0005769",
  "gene_name": "Sorting nexin-7"
}